regulation of JUN kinase activity [GO:0043506] (biological process) Relationships: is a type of regulation of MAP kinase activity [GO:0043405]; RO_0002211 JUN kinase activity [GO:0004705] Sources: GOC:jl Also known as: regulation of JUNK activity Subtypes: GO:0043507, negative regulation of JUN kinase activity [GO:0043508] Definition: Any process that modulates the frequency, rate or extent of JUN kinase activity.